{
  "gene": "UniProtKB:Q9BTZ2",
  "term_label": "carbonyl reductase (NADPH) activity",
  "gene_symbol": "DHRS4",
  "term_id": "GO:0004090",
  "gene_name": "Dehydrogenase_reductase SDR family member 4"
}